{
  "term_id": "GO:0042393",
  "gene": "UniProtKB:O14646",
  "term_label": "histone binding",
  "gene_symbol": "CHD1",
  "gene_name": "Chromodomain-helicase-DNA-binding protein 1"
}